{
  "gene_name": "Amiloride-sensitive sodium channel subunit gamma",
  "gene": "UniProtKB:P51170",
  "term_id": "GO:0034706",
  "term_label": "sodium channel complex",
  "gene_symbol": "SCNN1G"
}